{
  "term_label": "calcium/calmodulin-dependent protein kinase activity",
  "gene_name": "MAP kinase-activated protein kinase 2",
  "gene": "UniProtKB:P49137",
  "term_id": "GO:0004683",
  "gene_symbol": "MAPKAPK2"
}